{
  "gene_name": "Relaxin receptor 2",
  "term_label": "G protein-coupled peptide receptor activity",
  "gene_symbol": "RXFP2",
  "gene": "UniProtKB:Q8WXD0",
  "term_id": "GO:0008528"
}